RecQ family helicase-topoisomerase III complex [GO:0031422] (cellular component) References: PMID:15889139 Sources: GOC:bhm, GOC:krc Relationships: is a type of DNA helicase complex [GO:0033202]; is part of chromosome [GO:0005694] Definition: A complex containing a RecQ family helicase and a topoisomerase III homologue (a member of the topoisomerase type IA subfamily); may also include one or more additional proteins; conserved from E. coli to human. Also known as: RecQ helicase-Topo III complex, Sgs1-Top3 complex